CD4-positive, alpha-beta T cell differentiation [GO:0043367] (biological process) Note: Note that immunologists typically use the word 'development' to refer to cells of B or T cell lineages undergoing the process that GO describes as 'cell differentiation'. Relationships: is a type of GO:0035710; is a type of GO:0046632 Subtypes: GO:0002294, GO:0002301, CD4-positive, CD25-positive, alpha-beta regulatory T cell differentiation [GO:0002361] Also known as: CD4-positive, alpha beta T cell differentiation, CD4-positive, alpha-beta T lymphocyte differentiation, CD4-positive, alpha-beta T-cell differentiation, CD4-positive, alpha-beta T-lymphocyte differentiation, CD4-positive, alpha beta T cell development Sources: CL:0000624, ISBN:0781735149 Regulation: regulated by regulation of CD4-positive, alpha-beta T cell differentiation [GO:0043370]; negatively regulated by GO:0043371; positively regulated by GO:0043372 Definition: The process in which a relatively unspecialized T cell acquires specialized features of a mature CD4-positive, alpha-beta T cell.